{
  "term_id": "GO:0048476",
  "gene": "UniProtKB:Q96NY9",
  "gene_symbol": "MUS81",
  "term_label": "Holliday junction resolvase complex",
  "gene_name": "Crossover junction endonuclease MUS81"
}